{
  "gene": "UniProtKB:O00743",
  "term_label": "protein serine/threonine phosphatase activity",
  "term_id": "GO:0004722",
  "gene_symbol": "PPP6C",
  "gene_name": "Serine_threonine-protein phosphatase 6 catalytic subunit"
}